{
  "term_id": "UNKNOWN:0002",
  "term_label": "Unknown biological process",
  "gene_name": "Membrane protein BRI3",
  "gene_symbol": "BRI3",
  "gene": "UniProtKB:O95415"
}